{
  "term_label": "plasma membrane",
  "gene": "UniProtKB:Q9NR97",
  "gene_symbol": "TLR8",
  "term_id": "GO:0005886",
  "gene_name": "Toll-like receptor 8"
}